{
  "gene_name": "Uncharacterized protein C3orf85",
  "gene_symbol": "C3orf85",
  "gene": "UniProtKB:A0A1B0GTC6",
  "term_id": "UNKNOWN:0003",
  "term_label": "Unknown cellular component"
}